{
  "gene_symbol": "IGKJ2",
  "gene": "UniProtKB:A0A0A0MT85",
  "gene_name": "Immunoglobulin kappa joining 2 (Fragment)",
  "term_label": "Unknown cellular component",
  "term_id": "UNKNOWN:0003"
}